{
  "term_id": "GO:0051145",
  "gene_symbol": "MRTFB",
  "term_label": "smooth muscle cell differentiation",
  "gene_name": "Myocardin-related transcription factor B",
  "gene": "UniProtKB:Q9ULH7"
}